{
  "gene_name": "Cyclic AMP-responsive element-binding protein 3-like protein 2",
  "gene": "UniProtKB:Q70SY1",
  "term_label": "cAMP response element binding",
  "gene_symbol": "CREB3L2",
  "term_id": "GO:0035497"
}